regulation of myofibroblast cell apoptotic process [GO:1904520] (biological process) Also known as: regulation of MFB apoptotic process, regulation of MFB apoptosis, regulation of myofibroblast cell apoptosis Relationships: is a type of regulation of apoptotic process [GO:0042981]; regulates GO:1904516 Definition: Any process that modulates the frequency, rate or extent of myofibroblast cell apoptotic process. Subtypes: negative regulation of myofibroblast cell apoptotic process [GO:1904521], positive regulation of myofibroblast cell apoptotic process [GO:1904522] References: PMID:26119034 Sources: GOC:TermGenie, GO_REF:0000058